{
  "gene_symbol": "SAMD9L",
  "gene": "UniProtKB:Q8IVG5",
  "gene_name": "Sterile alpha motif domain-containing protein 9-like",
  "term_label": "Unknown molecular function",
  "term_id": "UNKNOWN:0001"
}